{
  "gene_name": "Disintegrin and metalloproteinase domain-containing protein 28",
  "gene_symbol": "ADAM28",
  "gene": "UniProtKB:Q9UKQ2",
  "term_id": "GO:0005886",
  "term_label": "plasma membrane"
}